{
  "gene_name": "Cytochrome c oxidase assembly factor 5",
  "term_label": "mitochondrial respiratory chain complex IV assembly",
  "gene_symbol": "COA5",
  "term_id": "GO:0033617",
  "gene": "UniProtKB:Q86WW8"
}